{
  "gene": "UniProtKB:Q9Y2R9",
  "term_label": "structural constituent of ribosome",
  "gene_symbol": "MRPS7",
  "gene_name": "Small ribosomal subunit protein uS7m",
  "term_id": "GO:0003735"
}